nucleic acid catabolic process [GO:0141188] (biological process) Note: This term should not be used for direct annotation. It should be possible to make a more specific annotation to one of the children of this term. Subtypes: DNA catabolic process [GO:0006308], RNA catabolic process [GO:0006401] Sources: GOC:curators Definition: The cellular DNA metabolic process resulting in the breakdown of a nucleic acid. Relationships: is a type of GO:0009057; is a type of nucleobase-containing compound catabolic process [GO:0034655]; is a type of nucleic acid metabolic process [GO:0090304]